{
  "term_id": "GO:0000977",
  "gene_name": "Zinc finger protein 875",
  "gene": "UniProtKB:P10072",
  "term_label": "RNA polymerase II transcription regulatory region sequence-specific DNA binding",
  "gene_symbol": "ZNF875"
}